type 3 melanocortin receptor binding [GO:0031781] (molecular function) Definition: Binding to a type 3 melanocortin receptor. Sources: GOC:mah, GOC:nln Relationships: is a type of melanocortin receptor binding [GO:0031779] Also known as: type 3 melanocortin receptor ligand